anaphase [GO:0051322] (biological process) Subtypes: mitotic anaphase [GO:0000090] Note: Note that this term should not be used for direct annotation. If you are trying to make an annotation to x phase, it is likely that the correct annotation is 'regulation of x/y phase transition' or to a process which occurs during the reported phase (i.e mitotic DNA replication for mitotic S-phase). To capture the phase when a specific location or process is observed, the phase term can be used in an annotation extension (PMID:24885854) applied to a cellular component term (with the relation exists_during) or a biological process term (with the relation happens_during). Relationships: is a type of cell cycle phase [GO:0022403]; is part of M phase [GO:0000279] Definition: The cell cycle phase, following metaphase, during which the chromosomes separate and migrate towards the poles of the spindle. Sources: GOC:mtg_cell_cycle